{
  "gene": "UniProtKB:O15537",
  "term_id": "GO:0005615",
  "term_label": "extracellular space",
  "gene_name": "Retinoschisin",
  "gene_symbol": "RS1"
}